{
  "term_label": "chemical synaptic transmission",
  "term_id": "GO:0007268",
  "gene_name": "Spatacsin",
  "gene": "UniProtKB:Q96JI7",
  "gene_symbol": "SPG11"
}